negative regulation of striated muscle tissue development [GO:0045843] (biological process) Sources: GOC:go_curators Relationships: is_a GO:0016202; is a type of negative regulation of muscle organ development [GO:0048635]; is a type of negative regulation of muscle tissue development [GO:1901862]; negatively regulates striated muscle tissue development [GO:0014706] Definition: Any process that stops, prevents, or reduces the frequency, rate or extent of striated muscle development. Also known as: down regulation of striated muscle development, down-regulation of striated muscle development, downregulation of striated muscle development, inhibition of striated muscle development Subtypes: negative regulation of skeletal muscle tissue development [GO:0048642], GO:0055026